{
  "gene_name": "Protein reprimo",
  "gene": "UniProtKB:Q9NS64",
  "term_id": "UNKNOWN:0001",
  "term_label": "Unknown molecular function",
  "gene_symbol": "RPRM"
}